{
  "gene_symbol": "POTEA",
  "gene_name": "POTE ankyrin domain family member A",
  "term_id": "UNKNOWN:0001",
  "gene": "UniProtKB:Q6S8J7",
  "term_label": "Unknown molecular function"
}